Krueppel-associated box domain binding [GO:0035851] (molecular function) Relationships: is a type of GO:0019904 Sources: InterPro:IPR001909 Also known as: KRAB domain binding, Krueppel-associated box binding Definition: Binding to a Krueppel-associated box (KRAB) domain of a protein. The approximately 75 amino acid KRAB domain is enriched in charged amino acids, and is found in the N-terminal regions of many zinc finger-containing transcription factors.